{
  "gene": "UniProtKB:Q9UEU0",
  "term_id": "GO:0042147",
  "gene_name": "Vesicle transport through interaction with t-SNAREs homolog 1B",
  "gene_symbol": "VTI1B",
  "term_label": "retrograde transport, endosome to Golgi"
}